{
  "gene": "UniProtKB:Q9Y6W5",
  "term_label": "Arp2/3 complex binding",
  "gene_name": "Actin-binding protein WASF2",
  "term_id": "GO:0071933",
  "gene_symbol": "WASF2"
}